{
  "term_label": "digestive tract development",
  "gene": "UniProtKB:Q9HCK8",
  "term_id": "GO:0048565",
  "gene_symbol": "CHD8",
  "gene_name": "Chromodomain-helicase-DNA-binding protein 8"
}